regulation of vesicle fusion with Golgi apparatus [GO:0106214] (biological process) References: PMID:26195667 Sources: GOC:se Definition: Any process that modulates the frequency, rate or extent of vesicle fusion with Golgi apparatus. Subtypes: negative regulation of vesicle fusion with Golgi apparatus [GO:0106215], GO:0106216 Relationships: is_a regulation of vesicle fusion [GO:0031338]; is a type of GO:1903358; regulates vesicle fusion with Golgi apparatus [GO:0048280]